regulation of smoothened signaling pathway [GO:0008589] (biological process) Also known as: regulation of hedgehog signaling pathway, regulation of hh signaling pathway, regulation of smoothened signalling pathway, regulation of smoothened activity, regulation of smoothened by patched, regulation of smoothened receptor activity by patched Sources: GOC:go_curators Definition: Any process that modulates the frequency, rate or extent of smoothened signaling. Subtypes: negative regulation of smoothened signaling pathway [GO:0045879], positive regulation of smoothened signaling pathway [GO:0045880], regulation of smoothened signaling pathway involved in dorsal/ventral neural tube patterning [GO:1901620] Relationships: is a type of regulation of signal transduction [GO:0009966]; regulates smoothened signaling pathway [GO:0007224]